endothelial cell activation within high endothelial venule involved in immune response [GO:0002259] (biological process) Definition: A change in the morphology or behavior of an endothelial cell within a high endothelial venule resulting from exposure to an activating factor such as a cellular or soluble ligand, leading to the initiation or perpetuation of an immune response. Also known as: endothelial cell activation within high endothelial venule during immune response Sources: GOC:add, ISBN:0781735149 Relationships: is_a endothelial cell activation involved in immune response [GO:0002264]